{
  "term_label": "endosome",
  "gene": "UniProtKB:O75129",
  "gene_symbol": "ASTN2",
  "gene_name": "Astrotactin-2",
  "term_id": "GO:0005768"
}